positive regulation of cell cycle G2/M phase transition [GO:1902751] (BP) Subtypes: positive regulation of G2/M transition of mitotic cell cycle [GO:0010971], positive regulation of G2/MI transition of meiotic cell cycle [GO:0110032] Sources: GOC:TermGenie, GOC:jl, GO_REF:0000058 Definition: Any signaling pathway that activates or increases the activity of a cell cycle cyclin-dependent protein kinase to modulate the switch from G2 phase to M phase of the cell cycle. Also known as: up regulation of cell cycle G2/M phase transition, up-regulation of cell cycle G2/M phase transition, upregulation of cell cycle G2/M phase transition, activation of cell cycle G2/M phase transition Relationships: is a type of positive regulation of cell cycle phase transition [GO:1901989]; is_a regulation of cell cycle G2/M phase transition [GO:1902749]; positively regulates cell cycle G2/M phase transition [GO:0044839]